{
  "gene": "UniProtKB:Q14765",
  "term_id": "GO:0006952",
  "term_label": "defense response",
  "gene_name": "Signal transducer and activator of transcription 4",
  "gene_symbol": "STAT4"
}